{
  "gene_symbol": "GTF3C1",
  "term_id": "GO:0000127",
  "gene": "UniProtKB:Q12789",
  "term_label": "transcription factor TFIIIC complex",
  "gene_name": "General transcription factor 3C polypeptide 1"
}